{
  "term_id": "GO:0048007",
  "term_label": "antigen processing and presentation, exogenous lipid antigen via MHC class Ib",
  "gene_symbol": "CD1C",
  "gene_name": "T-cell surface glycoprotein CD1c",
  "gene": "UniProtKB:P29017"
}